{
  "term_id": "GO:0005634",
  "gene": "UniProtKB:Q02539",
  "term_label": "nucleus",
  "gene_symbol": "H1-1",
  "gene_name": "Histone H1.1"
}